{
  "term_label": "tumor necrosis factor receptor binding",
  "term_id": "GO:0005164",
  "gene_name": "TNF receptor-associated factor 2",
  "gene_symbol": "TRAF2",
  "gene": "UniProtKB:Q12933"
}